epidermis morphogenesis [GO:0048730] (biological process) Definition: The process in which the anatomical structures of the epidermis are generated and organized. The epidermis is the outer epithelial layer of an animal, it may be a single layer that produces an extracellular material (e.g. the cuticle of arthropods) or a complex stratified squamous epithelium, as in the case of many vertebrate species. Sources: GOC:jid, UBERON:0001003 Also known as: hypodermis morphogenesis Relationships: is a type of morphogenesis of an epithelium [GO:0002009]; is part of epidermis development [GO:0008544] Subtypes: epidermis morphogenesis involved in nipple formation [GO:0060660]